{
  "term_id": "GO:0006183",
  "gene": "UniProtKB:P20839",
  "term_label": "GTP biosynthetic process",
  "gene_symbol": "IMPDH1",
  "gene_name": "Inosine-5'-monophosphate dehydrogenase 1"
}